positive regulation of penile erection [GO:0060406] (biological process) Relationships: is a type of positive regulation of multicellular organismal process [GO:0051240]; is a type of regulation of penile erection [GO:0060405]; is a type of GO:2000243; positively regulates GO:0043084 Sources: GOC:dph, GOC:tb Definition: Any process that increases the rate, frequency or extent of penile erection. Penile erection is the hardening, enlarging and rising of the penis which often occurs in the sexually aroused male and enables sexual intercourse. Achieved by increased inflow of blood into the vessels of erectile tissue, and decreased outflow.